{
  "gene": "UniProtKB:Q99717",
  "term_label": "BMP signaling pathway",
  "gene_symbol": "SMAD5",
  "term_id": "GO:0030509",
  "gene_name": "Mothers against decapentaplegic homolog 5"
}